pronephric proximal tubule morphogenesis [GO:0039011] (biological process) Definition: The process in which the anatomical structures of a pronephric nephron proximal tubule are generated and organized. A pronephric nephron tubule is an epithelial tube that is part of the pronephros. Relationships: is_a pronephric nephron tubule morphogenesis [GO:0039008]; is_a GO:0072158; is part of pronephric proximal tubule development [GO:0035776] Also known as: pronephros proximal tubule morphogenesis Sources: GOC:mtg_kidney_jan10